{
  "term_label": "protein monoubiquitination",
  "gene_symbol": "PEX12",
  "gene": "UniProtKB:O00623",
  "term_id": "GO:0006513",
  "gene_name": "Peroxisome assembly protein 12"
}